alpha-tubulin acetylation [GO:0071929] (biological process) Definition: The addition of an acetyl group to the lysine 40 residue of alpha-tubulin. References: PMID:17786050 Sources: GOC:kmv Relationships: is_a internal peptidyl-lysine acetylation [GO:0018393]